negative regulation of C-C chemokine receptor CCR7 signaling pathway [GO:1903081] (biological process) Relationships: is a type of negative regulation of chemokine-mediated signaling pathway [GO:0070100]; is a type of regulation of C-C chemokine receptor CCR7 signaling pathway [GO:1903080]; negatively regulates C-C chemokine receptor CCR7 signaling pathway [GO:0038118] Definition: Any process that stops, prevents or reduces the frequency, rate or extent of C-C chemokine receptor CCR7 signaling pathway. References: PMID:11602640 Sources: GOC:BHF, GOC:TermGenie, GOC:rl, GO_REF:0000058 Also known as: down regulation of C-C chemokine receptor CCR7 signaling pathway, down regulation of C-C chemokine receptor CCR7 signalling pathway, down-regulation of C-C chemokine receptor CCR7 signaling pathway, down-regulation of C-C chemokine receptor CCR7 signalling pathway, downregulation of C-C chemokine receptor CCR7 signaling pathway, downregulation of C-C chemokine receptor CCR7 signalling pathway, negative regulation of C-C chemokine receptor CCR7 signalling pathway, inhibition of C-C chemokine receptor CCR7 signaling pathway, inhibition of C-C chemokine receptor CCR7 signalling pathway, down regulation of CCR7 signaling pathway, down-regulation of CCR7 signaling pathway, downregulation of CCR7 signaling pathway, inhibition of CCR7 signaling pathway, negative regulation of CCR7 signaling pathway